{
  "gene_name": "Calmodulin-like protein 4",
  "gene_symbol": "CALML4",
  "term_id": "GO:0000226",
  "term_label": "microtubule cytoskeleton organization",
  "gene": "UniProtKB:Q96GE6"
}